negative regulation of trichome patterning [GO:1900033] (biological process) Definition: Any process that stops, prevents or reduces the frequency, rate or extent of trichome patterning. Relationships: is_a GO:0010648; is a type of negative regulation of signaling [GO:0023057]; is a type of negative regulation of multicellular organismal process [GO:0051241]; is a type of regulation of trichome patterning [GO:1900032]; negatively regulates trichome patterning [GO:0048629] Sources: GOC:TermGenie Also known as: down regulation of trichome distribution, down-regulation of trichome distribution, downregulation of trichome distribution, inhibition of trichome distribution, negative regulation of trichome distribution, down regulation of trichome pattern biosynthesis, down regulation of trichome pattern formation, down regulation of trichome spacing, down-regulation of trichome pattern biosynthesis, down-regulation of trichome pattern formation, down-regulation of trichome spacing, downregulation of trichome pattern biosynthesis, downregulation of trichome pattern formation, downregulation of trichome spacing, inhibition of trichome pattern biosynthesis, inhibition of trichome pattern formation, inhibition of trichome spacing, negative regulation of trichome pattern biosynthesis, negative regulation of trichome pattern formation, negative regulation of trichome spacing, down regulation of trichome pattern specification, down regulation of trichome patterning, down-regulation of trichome pattern specification, down-regulation of trichome patterning, downregulation of trichome pattern specification, downregulation of trichome patterning, inhibition of trichome pattern specification, inhibition of trichome patterning, negative regulation of trichome pattern specification